{
  "gene": "UniProtKB:Q9UBV8",
  "gene_symbol": "PEF1",
  "term_label": "Unknown molecular function",
  "term_id": "UNKNOWN:0001",
  "gene_name": "Peflin"
}